{
  "gene": "UniProtKB:Q9Y519",
  "term_label": "transmembrane transporter activity",
  "gene_symbol": "TMEM184B",
  "gene_name": "Transmembrane protein 184B",
  "term_id": "GO:0022857"
}